{
  "term_id": "GO:0002767",
  "gene_name": "Killer cell immunoglobulin-like receptor 2DL5B",
  "term_label": "immune response-inhibiting cell surface receptor signaling pathway",
  "gene_symbol": "KIR2DL5B",
  "gene": "UniProtKB:Q8NHK3"
}